{
  "gene_symbol": "WNT9A",
  "term_label": "frizzled binding",
  "gene": "UniProtKB:O14904",
  "gene_name": "Protein Wnt-9a",
  "term_id": "GO:0005109"
}